{
  "gene_name": "Glutathione S-transferase theta-4",
  "term_id": "GO:0005737",
  "term_label": "cytoplasm",
  "gene": "UniProtKB:A0A1W2PR19",
  "gene_symbol": "GSTT4"
}